{
  "gene": "UniProtKB:Q9Y4C1",
  "gene_symbol": "KDM3A",
  "gene_name": "Lysine-specific demethylase 3A",
  "term_id": "GO:0032454",
  "term_label": "histone H3K9 demethylase activity"
}